{
  "gene_symbol": "MCRIP1",
  "term_id": "UNKNOWN:0003",
  "gene_name": "Mapk-regulated corepressor-interacting protein 1",
  "gene": "UniProtKB:C9JLW8",
  "term_label": "Unknown cellular component"
}